{
  "term_label": "extracellular space",
  "gene": "UniProtKB:P10643",
  "term_id": "GO:0005615",
  "gene_symbol": "C7",
  "gene_name": "Complement component C7"
}